glutamine transport [GO:0006868] (BP) Also known as: L-glutamine transport Definition: The directed movement of glutamine, 2-amino-4-carbamoylbutanoic acid, into, out of or within a cell, or between cells, by means of some agent such as a transporter or pore. Subtypes: glutamine secretion [GO:0010585], L-glutamine import across plasma membrane [GO:1903803] Regulation: regulated by regulation of glutamine transport [GO:2000485]; negatively regulated by negative regulation of glutamine transport [GO:2000486]; positively regulated by GO:2000487 Relationships: is a type of GO:0015804; is a type of carboxylic acid transport [GO:0046942]; is a type of nitrogen compound transport [GO:0071705] Sources: GOC:ai